Malpighian tubule development [GO:0072002] (biological process) Definition: The process whose specific outcome is the progression of the Malpighian tubule over time, from its formation to the mature structure. A Malpighian tubule is a fine, thin-walled excretory tubule in insects which leads into the posterior part of the gut. References: PMID:19783135 Sources: FBbt:00005786, GOC:mtg_kidney_jan10 Relationships: is a type of animal organ development [GO:0048513]; is a type of GO:0061326 Subtypes: anterior Malpighian tubule development [GO:0061327], posterior Malpighian tubule development [GO:0061328]